{
  "term_id": "UNKNOWN:0002",
  "term_label": "Unknown biological process",
  "gene_symbol": "A0A804HJP8",
  "gene_name": "Uncharacterized protein",
  "gene": "UniProtKB:A0A804HJP8"
}